{
  "term_label": "N-glycan processing",
  "gene_name": "Beta-hexosaminidase subunit beta",
  "term_id": "GO:0006491",
  "gene": "UniProtKB:P07686",
  "gene_symbol": "HEXB"
}